{
  "gene_name": "Protein numb homolog",
  "term_id": "UNKNOWN:0001",
  "term_label": "Unknown molecular function",
  "gene": "UniProtKB:P49757",
  "gene_symbol": "NUMB"
}